{
  "gene_symbol": "SOX12",
  "gene": "UniProtKB:O15370",
  "term_id": "GO:0005634",
  "gene_name": "Transcription factor SOX-12",
  "term_label": "nucleus"
}